{
  "gene": "UniProtKB:Q7RTV0",
  "gene_symbol": "PHF5A",
  "gene_name": "PHD finger-like domain-containing protein 5A",
  "term_label": "Unknown molecular function",
  "term_id": "UNKNOWN:0001"
}